{
  "term_id": "GO:0045892",
  "term_label": "negative regulation of DNA-templated transcription",
  "gene": "UniProtKB:Q96NU1",
  "gene_name": "Sterile alpha motif domain-containing protein 11",
  "gene_symbol": "SAMD11"
}